somatic diversification of immunoglobulin genes by N region addition [GO:0002570] (biological process) Definition: The addition of variable numbers of random nucleotides by terminal deoxytransferase in the N regions of heavy chain immunoglobulin genes. N regions are found at the V-D and D-J recombinational junctions. Relationships: is a type of somatic diversification of immune receptors by N region addition [GO:0002569]; is a type of somatic diversification of immunoglobulins [GO:0016445]; is part of somatic recombination of immunoglobulin gene segments [GO:0016447] Sources: GOC:add, ISBN:0781735149 Also known as: somatic diversification of antibody genes by N region addition